{
  "gene_name": "Proline-rich protein 15-like protein",
  "term_id": "UNKNOWN:0002",
  "gene_symbol": "PRR15L",
  "term_label": "Unknown biological process",
  "gene": "UniProtKB:Q9BU68"
}